somatic muscle development [GO:0007525] (biological process) Subtypes: larval somatic muscle development [GO:0007526], adult somatic muscle development [GO:0007527], somatic muscle attachment to chitin-based cuticle [GO:0160175] Sources: GOC:jid, GOC:mtg_muscle Relationships: is a type of muscle structure development [GO:0061061] Definition: The process whose specific outcome is the progression of the somatic muscle over time, from its formation to the mature structure. Somatic muscles are striated muscle structures that connect to the exoskeleton or cuticle. Regulation: regulated by regulation of somatic muscle development [GO:0062223]; positively regulated by positive regulation of somatic muscle development [GO:0062224]; negatively regulated by GO:0062225